{
  "term_label": "cell surface",
  "term_id": "GO:0009986",
  "gene_name": "T-cell immunoreceptor with Ig and ITIM domains",
  "gene": "UniProtKB:Q495A1",
  "gene_symbol": "TIGIT"
}